gamma-glutamyl hercynylcysteine sulfoxide synthase activity [GO:0044875] (molecular function) References: PMID:24828577 Sources: GOC:jl, RHEA:42672 Relationships: is a type of GO:0004497; is a type of GO:0016705; is part of ergothioneine biosynthesis from histidine via gamma-glutamyl-hercynylcysteine sulfoxide [GO:0052704] Definition: Catalysis of the reaction: gamma-glutamyl cysteine + hercynine + O2 = gamma-glutamyl-hercynyl cysteine sulfoxide + H2O. Also known as: gamma-glutamyl hercynylcysteine S-oxide synthase, gamma-glutamyl hercynylcysteine sulfoxide synthase